{
  "gene_symbol": "HSPA12A",
  "term_id": "UNKNOWN:0003",
  "gene": "UniProtKB:O43301",
  "gene_name": "Heat shock 70 kDa protein 12A",
  "term_label": "Unknown cellular component"
}